{
  "term_id": "GO:0007399",
  "gene": "UniProtKB:Q9GZZ7",
  "gene_symbol": "GFRA4",
  "term_label": "nervous system development",
  "gene_name": "GDNF family receptor alpha-4"
}